{
  "gene": "UniProtKB:O43490",
  "gene_symbol": "PROM1",
  "gene_name": "Prominin-1",
  "term_label": "microvillus",
  "term_id": "GO:0005902"
}